regulation of female gonad development [GO:2000194] (biological process) Also known as: regulation of ovarian development, regulation of ovary development Subtypes: negative regulation of female gonad development [GO:2000195], positive regulation of female gonad development [GO:2000196], regulation of progesterone secretion [GO:2000870] Definition: Any process that modulates the frequency, rate or extent of female gonad development. Sources: GOC:obol Relationships: is a type of GO:1905939; is a type of regulation of multicellular organismal development [GO:2000026]; regulates GO:0008585